{
  "gene_symbol": "SDC2",
  "term_label": "cell surface",
  "term_id": "GO:0009986",
  "gene_name": "Syndecan-2",
  "gene": "UniProtKB:P34741"
}